{
  "gene_name": "Protein FAM149A",
  "term_id": "UNKNOWN:0002",
  "term_label": "Unknown biological process",
  "gene": "UniProtKB:A5PLN7",
  "gene_symbol": "FAM149A"
}